{
  "gene_name": "Tyrosine-protein kinase Mer",
  "term_label": "plasma membrane",
  "term_id": "GO:0005886",
  "gene": "UniProtKB:Q12866",
  "gene_symbol": "MERTK"
}